post-embryonic plant morphogenesis [GO:0090698] (biological process) Definition: The process, occurring after plant embryonic development, by which anatomical structures are generated and organized. Subtypes: stomatal complex morphogenesis [GO:0010103], guard cell morphogenesis [GO:0010442], inflorescence morphogenesis [GO:0048281], GO:0048317, flower morphogenesis [GO:0048439], floral whorl morphogenesis [GO:0048457], plant ovule morphogenesis [GO:0048482], fruit morphogenesis [GO:0048530], anther wall tapetum morphogenesis [GO:0048655], cotyledon morphogenesis [GO:0048826], post-embryonic plant organ morphogenesis [GO:0090697] Sources: GOC:tb Relationships: is a type of anatomical structure morphogenesis [GO:0009653]